{
  "gene": "UniProtKB:Q9Y278",
  "gene_symbol": "HS3ST2",
  "term_id": "UNKNOWN:0002",
  "gene_name": "Heparan sulfate glucosamine 3-O-sulfotransferase 2",
  "term_label": "Unknown biological process"
}